{
  "gene_name": "Protocadherin alpha-10",
  "term_id": "GO:0007155",
  "term_label": "cell adhesion",
  "gene_symbol": "PCDHA10",
  "gene": "UniProtKB:Q9Y5I2"
}